{
  "term_id": "GO:0016477",
  "gene": "UniProtKB:Q9NQT6",
  "gene_name": "Fascin-3",
  "gene_symbol": "FSCN3",
  "term_label": "cell migration"
}